{
  "term_label": "Unknown molecular function",
  "gene_name": "Putative uncharacterized protein SSBP3-AS1",
  "gene": "UniProtKB:Q7Z2R9",
  "gene_symbol": "SSBP3-AS1",
  "term_id": "UNKNOWN:0001"
}